{
  "term_id": "UNKNOWN:0002",
  "gene": "UniProtKB:Q9H611",
  "gene_symbol": "PIF1",
  "gene_name": "ATP-dependent DNA helicase PIF1",
  "term_label": "Unknown biological process"
}